{
  "gene": "UniProtKB:P41567",
  "gene_symbol": "EIF1",
  "gene_name": "Eukaryotic translation initiation factor 1",
  "term_id": "GO:0016282",
  "term_label": "eukaryotic 43S preinitiation complex"
}